{
  "gene_name": "Unconventional myosin-IXb",
  "term_label": "ruffle",
  "term_id": "GO:0001726",
  "gene": "UniProtKB:Q13459",
  "gene_symbol": "MYO9B"
}